L-arabinonate dehydratase activity [GO:0050020] (molecular function) Also known as: L-arabinonate hydro-lyase (2-dehydro-3-deoxy-L-arabinonate-forming), L-arabinonate hydro-lyase activity, L-arabonate dehydrase activity, L-arabonate dehydratase activity Relationships: is a type of hydro-lyase activity [GO:0016836] Definition: Catalysis of the reaction: L-arabinonate = 2-dehydro-3-deoxy-L-arabinonate + H2O. Sources: EC:4.2.1.25, RHEA:20968